{
  "gene_symbol": "HMX2",
  "term_label": "DNA-binding transcription factor activity, RNA polymerase II-specific",
  "term_id": "GO:0000981",
  "gene_name": "Homeobox protein HMX2",
  "gene": "UniProtKB:A2RU54"
}